endoplasmic reticulum membrane organization [GO:0090158] (biological process) Definition: A process that is carried out at the cellular level which results in the assembly, arrangement of constituent parts, or disassembly of an endoplasmic reticulum membrane. Subtypes: endoplasmic reticulum membrane fusion [GO:0016320], GO:1990809 Also known as: endoplasmic reticulum membrane organisation Relationships: is a type of membrane organization [GO:0061024]; is part of endoplasmic reticulum organization [GO:0007029] Sources: GOC:ascb_2009, GOC:dph, GOC:tb